detection of sucrose stimulus [GO:0009731] (biological process) Definition: The series of events in which a sucrose stimulus is received by a cell and converted into a molecular signal. Sources: GOC:sm Also known as: perception of sucrose stimulus Relationships: is a type of response to sucrose [GO:0009744]; is a type of detection of disaccharide stimulus [GO:0034288]